positive regulation of tissue kallikrein-kinin cascade [GO:0002547] (biological process) Definition: Any process that activates or increases the frequency, rate, or extent of the tissue kallikrein-kinin cascade. Relationships: is a type of positive regulation of kinin cascade [GO:0002258]; is a type of GO:0002382; positively regulates tissue kallikrein-kinin cascade [GO:0002255] Also known as: positive regulation of glandular kallikrein-kinin cascade, up regulation of tissue kallikrein-kinin cascade, up-regulation of tissue kallikrein-kinin cascade, upregulation of tissue kallikrein-kinin cascade, activation of tissue kallikrein-kinin cascade, stimulation of tissue kallikrein-kinin cascade Sources: GOC:add